{
  "gene_symbol": "GABRR2",
  "term_id": "GO:1902476",
  "gene": "UniProtKB:P28476",
  "term_label": "chloride transmembrane transport",
  "gene_name": "Gamma-aminobutyric acid receptor subunit rho-2"
}